{
  "gene_symbol": "SLC6A4",
  "gene": "UniProtKB:P31645",
  "gene_name": "Sodium-dependent serotonin transporter",
  "term_id": "GO:0005335",
  "term_label": "serotonin:sodium:chloride symporter activity"
}